{
  "gene_symbol": "LARP1",
  "gene_name": "La-related protein 1",
  "gene": "UniProtKB:Q6PKG0",
  "term_id": "GO:0045727",
  "term_label": "positive regulation of translation"
}